branch elongation of an epithelium [GO:0060602] (biological process) Subtypes: bud outgrowth involved in lung branching [GO:0060447], GO:0060449, primary prostatic bud elongation [GO:0060516], GO:0060523, branch elongation involved in salivary gland morphogenesis [GO:0060667], GO:0060681, branch elongation involved in mammary gland duct branching [GO:0060751] Sources: GOC:dph Definition: The growth process in which a branch increases in length from its base to its tip. Relationships: is a type of axis elongation [GO:0003401]; BFO_0000050 morphogenesis of a branching epithelium [GO:0061138]